{
  "term_label": "plasma membrane",
  "gene_name": "Lysosome-associated membrane glycoprotein 5",
  "gene": "UniProtKB:Q9UJQ1",
  "term_id": "GO:0005886",
  "gene_symbol": "LAMP5"
}